regulation of pulmonary blood vessel remodeling [GO:1905109] (biological process) Definition: Any process that modulates the frequency, rate or extent of pulmonary blood vessel remodeling. Relationships: is a type of regulation of blood vessel remodeling [GO:0060312]; RO_0002211 GO:0101010 Also known as: regulation of pulmonary blood vessel remodelling Subtypes: GO:1905110, positive regulation of pulmonary blood vessel remodeling [GO:1905111] References: PMID:22161164 Sources: GOC:BHF, GOC:BHF_miRNA, GOC:TermGenie, GOC:bc, GO_REF:0000058